{
  "gene_name": "GTP-binding protein 2",
  "gene_symbol": "GTPBP2",
  "term_label": "Unknown cellular component",
  "term_id": "UNKNOWN:0003",
  "gene": "UniProtKB:Q9BX10"
}